{
  "term_id": "GO:0003682",
  "term_label": "chromatin binding",
  "gene_name": "Sex comb on midleg-like protein 4",
  "gene_symbol": "SCML4",
  "gene": "UniProtKB:Q8N228"
}